{
  "term_id": "GO:0010494",
  "gene_symbol": "PABPC4L",
  "term_label": "cytoplasmic stress granule",
  "gene": "UniProtKB:P0CB38",
  "gene_name": "Polyadenylate-binding protein 4-like"
}